{
  "gene_name": "Histone-lysine N-methyltransferase SETD7",
  "term_id": "GO:0045893",
  "gene_symbol": "SETD7",
  "gene": "UniProtKB:Q8WTS6",
  "term_label": "positive regulation of DNA-templated transcription"
}